{
  "term_label": "cell surface receptor signaling pathway",
  "term_id": "GO:0007166",
  "gene_symbol": "ADGRA1",
  "gene": "UniProtKB:Q86SQ6",
  "gene_name": "Adhesion G protein-coupled receptor A1"
}